{
  "gene": "UniProtKB:P51861",
  "gene_symbol": "CDR1",
  "gene_name": "Cerebellar degeneration-related antigen 1",
  "term_label": "Unknown molecular function",
  "term_id": "UNKNOWN:0001"
}